{
  "gene": "UniProtKB:P01733",
  "gene_symbol": "TRBV12-3",
  "term_label": "Unknown molecular function",
  "gene_name": "T cell receptor beta variable 12-3",
  "term_id": "UNKNOWN:0001"
}